{
  "gene_name": "Meiotic nuclear division protein 1 homolog",
  "term_label": "nucleus",
  "gene": "UniProtKB:Q9BWT6",
  "term_id": "GO:0005634",
  "gene_symbol": "MND1"
}